{
  "gene_name": "Tumor necrosis factor receptor superfamily member 1A",
  "term_label": "inflammatory response",
  "term_id": "GO:0006954",
  "gene": "UniProtKB:P19438",
  "gene_symbol": "TNFRSF1A"
}